{
  "gene_name": "EF-hand domain-containing protein D1",
  "term_label": "Unknown biological process",
  "gene": "UniProtKB:Q9BUP0",
  "term_id": "UNKNOWN:0002",
  "gene_symbol": "EFHD1"
}